{
  "gene": "UniProtKB:O43570",
  "term_label": "Unknown biological process",
  "term_id": "UNKNOWN:0002",
  "gene_name": "Carbonic anhydrase 12",
  "gene_symbol": "CA12"
}